{
  "gene_symbol": "ZNF785",
  "term_id": "GO:0005634",
  "term_label": "nucleus",
  "gene_name": "Zinc finger protein 785",
  "gene": "UniProtKB:A8K8V0"
}